{
  "gene_symbol": "CDX2",
  "gene": "UniProtKB:Q99626",
  "gene_name": "Homeobox protein CDX-2",
  "term_id": "GO:0009948",
  "term_label": "anterior/posterior axis specification"
}